collagen binding [GO:0005518] (molecular function) Subtypes: collagen V binding [GO:0070052], collagen binding involved in cell-matrix adhesion [GO:0098639] Relationships: is_a protein-containing complex binding [GO:0044877] Sources: GOC:ai, ISBN:0198506732 Definition: Binding to collagen, a group of fibrous proteins of very high tensile strength that form the main component of connective tissue in animals. Collagen is highly enriched in glycine (some regions are 33% glycine) and proline, occurring predominantly as 3-hydroxyproline (about 20%).